cytoplasmic side of late endosome membrane [GO:0098560] (cellular component) Note: In GO, 'external side' still refers to part of the membrane and does not refer to components beyond (outside of) the membrane. Definition: The side (leaflet) of the late endosome membrane that faces the cytoplasm. Relationships: is a type of cytoplasmic side of endosome membrane [GO:0010009]; is part of GO:0031902 Sources: GOC:lr Also known as: external leaflet of late endosome membrane, external side of late endosome membrane